{
  "gene": "UniProtKB:O14777",
  "term_id": "GO:0051315",
  "term_label": "attachment of mitotic spindle microtubules to kinetochore",
  "gene_symbol": "NDC80",
  "gene_name": "Kinetochore protein NDC80 homolog"
}